{
  "gene_symbol": "CD24",
  "term_label": "cell activation",
  "term_id": "GO:0001775",
  "gene_name": "Signal transducer CD24",
  "gene": "UniProtKB:P25063"
}